negative regulation of telomere maintenance via semi-conservative replication [GO:0032214] (biological process) Also known as: down regulation of telomere maintenance via semi-conservative replication, down-regulation of telomere maintenance via semi-conservative replication, downregulation of telomere maintenance via semi-conservative replication, inhibition of telomere maintenance via semi-conservative replication Definition: Any process that stops, prevents, or reduces the frequency, rate or extent of the semi-conservative replication of telomeric DNA. Sources: GOC:mah Relationships: is a type of negative regulation of cell cycle process [GO:0010948]; is_a negative regulation of telomere maintenance [GO:0032205]; is a type of GO:0032213; negatively regulates telomere maintenance via semi-conservative replication [GO:0032201]